temperature-gated ion channel activity [GO:0097603] (molecular function) References: PMID:23027824 Sources: GOC:ha, GOC:pr Subtypes: temperature-gated cation channel activity [GO:0097604] Relationships: is a type of monoatomic ion channel activity [GO:0005216]; is a type of gated channel activity [GO:0022836] Definition: Enables the transmembrane transfer of an ion by a channel that opens in response to a temperature stimulus (e.g. exposure to a temperature range different than the optimal temperature for that organism). Also known as: temperature gated ion channel activity, temperature-activated ion channel activity, temperature-dependent ion channel activity, heat-activated ion channel activity